regulation of SA node cell action potential [GO:0098907] (biological process) Relationships: is a type of regulation of cell communication [GO:0010646]; is a type of regulation of cardiac muscle cell action potential [GO:0098901]; regulates SA node cell action potential [GO:0086015] Definition: Any process that modulates the frequency, rate or extent of action potential creation, propagation or termination in an SA node cardiac myocyte. This typically occurs via modulation of the activity or expression of voltage-gated ion channels. Sources: GOC:BHF, GOC:mtg_cardiac_conduct_nov11 Also known as: regulation of SA node cardiac muscle cell action potential, regulation of SAN cardiac muscle cell action potential, regulation of sinoatrial node cardiac muscle cell action potential, regulation of sinus node cardiac muscle cell action potential